{
  "gene": "UniProtKB:Q4G0N4",
  "gene_name": "NAD kinase 2, mitochondrial",
  "gene_symbol": "NADK2",
  "term_id": "GO:0019674",
  "term_label": "NAD+ metabolic process"
}